{
  "gene_symbol": "HTR5A",
  "term_id": "GO:0004993",
  "gene": "UniProtKB:P47898",
  "term_label": "G protein-coupled serotonin receptor activity",
  "gene_name": "5-hydroxytryptamine receptor 5A"
}